{
  "gene_symbol": "CAMKK1",
  "gene_name": "Calcium_calmodulin-dependent protein kinase kinase 1",
  "term_id": "GO:0004683",
  "term_label": "calcium/calmodulin-dependent protein kinase activity",
  "gene": "UniProtKB:Q8N5S9"
}